cell proliferation involved in atrial ventricular junction remodeling [GO:0003295] (biological process) Definition: The multiplication or reproduction of cells that contributes to the reorganization of tissue resulting in the maturation of the atrial ventricular junction. Sources: GOC:mtg_heart Also known as: cell proliferation involved in atrial ventricular junction remodelling, cell proliferation involved in atrio-ventricular junction remodeling, cell proliferation involved in atrio-ventricular junction remodelling, cell proliferation involved in atrioventricular junction remodeling, cell proliferation involved in atrioventricular junction remodelling Relationships: is a type of GO:0061323; is part of atrial ventricular junction remodeling [GO:0003294]